endodermal cell fate commitment [GO:0001711] (biological process) Relationships: is a type of cell fate commitment involved in formation of primary germ layer [GO:0060795]; is part of endodermal cell differentiation [GO:0035987] Also known as: endoderm cell fate commitment Definition: The cell differentiation process that results in commitment of a cell to become part of the endoderm. Sources: GOC:go_curators, ISBN:0878932437